{
  "term_label": "DNA methylation-dependent constitutive heterochromatin formation",
  "gene": "UniProtKB:A6NE82",
  "gene_symbol": "MBD3L3",
  "gene_name": "Putative methyl-CpG-binding domain protein 3-like 3",
  "term_id": "GO:0006346"
}